ATP transport [GO:0015867] (biological process) Definition: The directed movement of ATP, adenosine triphosphate, into, out of or within a cell, or between cells, by means of some agent such as a transporter or pore. Subtypes: GO:1904669, GO:1990544 Sources: GOC:ai Relationships: is a type of organic anion transport [GO:0015711]; is a type of GO:0015868; is a type of adenine nucleotide transport [GO:0051503]